{
  "term_id": "GO:0090090",
  "gene_symbol": "AXIN1",
  "term_label": "negative regulation of canonical Wnt signaling pathway",
  "gene": "UniProtKB:O15169",
  "gene_name": "Axin-1"
}